chemotropism [GO:0043577] (biological process) References: PMID:10087613 Sources: GOC:jl Relationships: is_a tropism [GO:0009606]; is part of response to chemical [GO:0042221] Definition: The movement of an organism, or part of an organism, in response to an external chemical gradient, usually toward or away from it.